negative regulation of transcription by RNA polymerase V [GO:1904280] (biological process) Also known as: down regulation of transcription from RNA pol V promoter, down regulation of transcription from RNA polymerase V promoter, down-regulation of transcription from RNA pol V promoter, down-regulation of transcription from RNA polymerase V promoter, downregulation of transcription from RNA pol V promoter, downregulation of transcription from RNA polymerase V promoter, negative regulation of transcription from RNA pol V promoter, negative regulation of transcription from RNA polymerase V promoter, inhibition of transcription from RNA pol V promoter, inhibition of transcription from RNA polymerase V promoter Relationships: is a type of GO:0045892; is a type of regulation of transcription by RNA polymerase V [GO:1904279]; negatively regulates transcription by RNA polymerase V [GO:0001060] Definition: Any process that stops, prevents or reduces the frequency, rate or extent of transcription mediated by RNA polymerase V. References: PMID:24726328 Sources: GOC:TermGenie, GO_REF:0000058